regulation of tube architecture, open tracheal system [GO:0035152] (biological process) Subtypes: lumen formation, open tracheal system [GO:0035149], regulation of tube size, open tracheal system [GO:0035151], maintenance of epithelial integrity, open tracheal system [GO:0035160] Relationships: is a type of regulation of biological quality [GO:0065008]; is part of open tracheal system development [GO:0007424] Also known as: regulation of tracheal tube architecture References: PMID:14570584 Sources: GOC:mtg_sensu Definition: Ensuring that tracheal cells form and maintain tubular structures with the correct size and shape for their position in the network. This is essential for efficient flow of gases through the tracheal network.